{
  "gene": "UniProtKB:Q9NWS6",
  "term_label": "Unknown cellular component",
  "term_id": "UNKNOWN:0003",
  "gene_symbol": "FAM118A",
  "gene_name": "Protein FAM118A"
}